{
  "gene_symbol": "OR6N2",
  "gene_name": "Olfactory receptor 6N2",
  "term_id": "GO:0004984",
  "term_label": "olfactory receptor activity",
  "gene": "UniProtKB:Q8NGY6"
}